{
  "gene": "UniProtKB:Q05397",
  "term_label": "non-membrane spanning protein tyrosine kinase activity",
  "gene_name": "Focal adhesion kinase 1",
  "term_id": "GO:0004715",
  "gene_symbol": "PTK2"
}